{
  "term_id": "GO:0019852",
  "gene_name": "Glutathione S-transferase omega-2",
  "term_label": "L-ascorbic acid metabolic process",
  "gene": "UniProtKB:Q9H4Y5",
  "gene_symbol": "GSTO2"
}